{
  "term_label": "negative regulation of RIG-I signaling pathway",
  "term_id": "GO:0039536",
  "gene_symbol": "GPATCH3",
  "gene": "UniProtKB:Q96I76",
  "gene_name": "G patch domain-containing protein 3"
}